{
  "gene_symbol": "C4BPA",
  "term_id": "GO:0005886",
  "term_label": "plasma membrane",
  "gene": "UniProtKB:P04003",
  "gene_name": "C4b-binding protein alpha chain"
}